histone H3K18 deacetylase activity, NAD-dependent [GO:0097372] (MF) Relationships: is a type of histone deacetylase activity, NAD-dependent [GO:0017136]; is a type of histone H3K deacetylase activity [GO:0141050] Note: Comment: Note that the residue position corresponds to the canonical human H3 histone (UniProtKB:P84243); this residue is conserved across all eukaryotes. Residue 1 is the first residue following removal of the initiating Methionine (Met). Note that each histone is encoded by multiple genes, and sequences may vary across different genes within an organism. Also known as: NAD-dependent histone H3-K18 deacetylase activity, NAD-dependent histone H3K18 deacetylase activity, NAD-dependent histone deacetylase activity (H3-K18 specific) Definition: Catalysis of the reaction: histone H3 N6-acetyl-L-lysine (position 18) + NAD+ + H2O = histone H3 L-lysine (position 18) + 2''-O-acetyl-ADP-D-ribose + nicotinamide. This reaction transfers an acetyl group attached to a lysine residue in H3K18 to NAD, producing nicotinamide. References: PMID:22722849, PMID:28450737 Sources: GOC:sp